{
  "gene_symbol": "PDSS1",
  "gene_name": "All trans-polyprenyl-diphosphate synthase PDSS1",
  "term_id": "GO:0032476",
  "gene": "UniProtKB:Q5T2R2",
  "term_label": "polyprenyl diphosphate synthase complex"
}